{
  "gene_name": "Insulin-like growth factor 1 receptor",
  "term_label": "positive regulation of phosphatidylinositol 3-kinase/protein kinase B signal transduction",
  "gene": "UniProtKB:P08069",
  "gene_symbol": "IGF1R",
  "term_id": "GO:0051897"
}